{
  "term_label": "pyrimidine nucleobase transport",
  "gene_symbol": "SLC28A1",
  "gene_name": "Sodium_nucleoside cotransporter 1",
  "gene": "UniProtKB:O00337",
  "term_id": "GO:0015855"
}